{
  "gene_name": "Unhealthy ribosome biogenesis protein 2 homolog",
  "gene": "UniProtKB:Q14146",
  "term_label": "Unknown molecular function",
  "term_id": "UNKNOWN:0001",
  "gene_symbol": "URB2"
}